{
  "gene_name": "FACT complex subunit SPT16",
  "term_label": "regulation of DNA-templated transcription elongation",
  "gene_symbol": "SUPT16H",
  "term_id": "GO:0032784",
  "gene": "UniProtKB:Q9Y5B9"
}